{
  "gene": "UniProtKB:Q13885",
  "term_id": "GO:0005874",
  "gene_name": "Tubulin beta-2A chain",
  "term_label": "microtubule",
  "gene_symbol": "TUBB2A"
}